protein localization to photoreceptor outer segment [GO:1903546] (biological process) Relationships: is a type of protein localization to non-motile cilium [GO:0097499] References: PMID:11481257, PMID:21867699 Sources: GOC:TermGenie, GO_REF:0000087 Also known as: protein localisation in photoreceptor outer segment, protein localisation to photoreceptor outer segment, protein localization in photoreceptor outer segment Definition: A process in which a protein is transported to, or maintained in, a location within a photoreceptor outer segment.